histone H1 kinase activity [GO:0140190] (MF) Definition: Catalysis of the transfer of a phosphate group to a histone H1. Subtypes: histone H1-4S187 kinase activity [GO:0140191], histone H1-4S27 kinase activity [GO:0140197], histone H1-4S35 kinase activity [GO:0140198] Relationships: is a type of histone kinase activity [GO:0035173] References: PMID:21511733, PMID:21852232, PMID:33238524